{
  "gene_name": "Proline-rich protein 14",
  "gene_symbol": "PRR14",
  "term_id": "UNKNOWN:0001",
  "term_label": "Unknown molecular function",
  "gene": "UniProtKB:Q9BWN1"
}